{
  "gene_name": "Transmembrane protein 14C",
  "gene": "UniProtKB:Q9P0S9",
  "term_id": "GO:0031966",
  "term_label": "mitochondrial membrane",
  "gene_symbol": "TMEM14C"
}